{
  "gene": "UniProtKB:P0C0E4",
  "gene_name": "Ras-related protein Rab-40A-like",
  "gene_symbol": "RAB40AL",
  "term_id": "GO:0005886",
  "term_label": "plasma membrane"
}